{
  "gene_name": "Telomerase-binding protein EST1A",
  "term_label": "telomeric DNA binding",
  "term_id": "GO:0042162",
  "gene": "UniProtKB:Q86US8",
  "gene_symbol": "SMG6"
}